cell cycle G2/M phase transition [GO:0044839] (biological process) Definition: The cell cycle process by which a cell in G2 phase commits to M phase. Relationships: is a type of cell cycle phase transition [GO:0044770] Sources: GOC:jl, GOC:mtg_cell_cycle Subtypes: G2/M transition of mitotic cell cycle [GO:0000086], GO:0008315 Regulation: regulated by regulation of cell cycle G2/M phase transition [GO:1902749]; negatively regulated by GO:1902750; positively regulated by positive regulation of cell cycle G2/M phase transition [GO:1902751]